{
  "term_id": "GO:0006616",
  "term_label": "SRP-dependent cotranslational protein targeting to membrane, translocation",
  "gene": "UniProtKB:P61011",
  "gene_symbol": "SRP54",
  "gene_name": "Signal recognition particle subunit SRP54"
}